dihydronicotinamide riboside quinone reductase activity [GO:0001512] (molecular function) Definition: Catalysis of the reaction: 1-(beta-D-ribofuranosyl)-1,4-dihydronicotinamide + a quinone = 1-(beta-D-ribofuranosyl)nicotinamide + a hydroquinone. Relationships: is a type of oxidoreductase activity, acting on diphenols and related substances as donors [GO:0016679] Also known as: ribosyldihydronicotinamide dehydrogenase (quinone) activity, NRH:quinone oxidoreductase 2 activity, N-ribosyldihydronicotinamide dehydrogenase (quinone) activity, NQO2, NQO2 activity, QR2 activity, quinone reductase 2 activity Sources: RHEA:12364